cell cycle DNA replication initiation [GO:1902292] (biological process) Also known as: DNA replication initiation involved in cell cycle DNA replication, DNA-dependent DNA replication initiation involved in cell cycle DNA replication, DNA endoreduplication initiation involved in cell cycle DNA replication, DNA re-replication initiation involved in cell cycle DNA replication Subtypes: nuclear cell cycle DNA replication initiation [GO:1902315], bacterial-type DNA replication initiation [GO:1902328] Definition: Any DNA replication initiation that is involved in cell cycle DNA replication. Sources: GOC:TermGenie, GOC:mtg_cell_cycle Relationships: is a type of DNA replication initiation [GO:0006270]; is a type of cell cycle process [GO:0022402]; is part of cell cycle DNA replication [GO:0044786]